{
  "gene": "UniProtKB:Q14344",
  "gene_name": "Guanine nucleotide-binding protein subunit alpha-13",
  "gene_symbol": "GNA13",
  "term_id": "GO:0007266",
  "term_label": "Rho protein signal transduction"
}